cone retinal bipolar cell differentiation [GO:1904390] (biological process) Also known as: cone bipolar cell differentiation, retinal cone bipolar cell differentiation References: PMID:24123365 Sources: GOC:TermGenie, GO_REF:0000086 Relationships: is a type of retinal bipolar neuron differentiation [GO:0060040] Definition: The process in which a relatively unspecialized cell acquires the specialized features of a cone retinal bipolar cell.